{
  "gene_symbol": "TRDN",
  "gene_name": "Triadin",
  "term_id": "GO:0005886",
  "gene": "UniProtKB:Q13061",
  "term_label": "plasma membrane"
}